{
  "term_id": "GO:0007129",
  "gene": "UniProtKB:Q8N6L0",
  "gene_symbol": "KASH5",
  "gene_name": "Protein KASH5",
  "term_label": "homologous chromosome pairing at meiosis"
}